{
  "term_id": "GO:2000812",
  "gene": "UniProtKB:P58546",
  "gene_symbol": "MTPN",
  "gene_name": "Myotrophin",
  "term_label": "regulation of barbed-end actin filament capping"
}